cytoplasm to vacuole targeting by the Cvt pathway [GO:0032258] (biological process) Definition: A cytoplasm to vacuole targeting pathway that uses machinery common with autophagy. The Cvt vesicle is formed when the receptor protein, Atg19, binds to the complexes of the target protein (aminopeptidase or alpha-mannosidase homododecamers), forming the Cvt complex. Atg11 binds to Atg9 and transports the Cvt complex to the pre-autophagosome (PAS). The phagophore membrane expands around the Cvt complex (excluding bulk cytoplasm) forming the Cvt vesicle. This pathway is mostly observed in yeast. Regulation: regulated by regulation of protein localization by the Cvt pathway [GO:2001159] Relationships: is a type of GO:0006623; is a type of process utilizing autophagic mechanism [GO:0061919]; has part vacuolar protein processing [GO:0006624] References: PMID:12865942, PMID:15659643